olefin biosynthetic process [GO:1900674] (biological process) Regulation: regulated by regulation of olefin biosynthetic process [GO:1900911]; negatively regulated by negative regulation of olefin biosynthetic process [GO:1900912]; RO_0002213 by GO:1900913 Also known as: olefin anabolism, olefin biosynthesis, olefin formation, olefin synthesis Subtypes: alkene biosynthetic process [GO:0043450], GO:0043612, limonene biosynthetic process [GO:0046250], GO:1900879, GO:1901940 Relationships: is a type of hydrocarbon biosynthetic process [GO:0120251]; is a type of olefinic compound biosynthetic process [GO:0120255]; is a type of olefin metabolic process [GO:1900673] Definition: The chemical reactions and pathways resulting in the formation of olefin. Sources: GOC:TermGenie, GOC:mengo_curators